{
  "gene_symbol": "NFIC",
  "gene_name": "Nuclear factor 1 C-type",
  "term_id": "GO:0005634",
  "term_label": "nucleus",
  "gene": "UniProtKB:P08651"
}